{
  "term_label": "plasma membrane",
  "gene": "UniProtKB:P32942",
  "gene_name": "Intercellular adhesion molecule 3",
  "gene_symbol": "ICAM3",
  "term_id": "GO:0005886"
}